{
  "term_label": "Unknown cellular component",
  "term_id": "UNKNOWN:0003",
  "gene_name": "Zinc finger protein 512B",
  "gene": "UniProtKB:Q96KM6",
  "gene_symbol": "ZNF512B"
}